{
  "gene": "UniProtKB:O95007",
  "term_label": "detection of chemical stimulus involved in sensory perception of smell",
  "term_id": "GO:0050911",
  "gene_symbol": "OR6B1",
  "gene_name": "Olfactory receptor 6B1"
}